ribulose bisphosphate carboxylase complex assembly [GO:0110102] (biological process) Also known as: RuBisCO assembly Definition: The aggregation, arrangement and bonding together of a set of components to form a ribulose bisphosphate carboxylase complex. Relationships: is_a protein-containing complex assembly [GO:0065003] References: PMID:29396988, PMID:29589905 Sources: GOC:krc, GOC:tb